{
  "gene_symbol": "RYR2",
  "gene": "UniProtKB:Q92736",
  "term_id": "GO:0014808",
  "term_label": "release of sequestered calcium ion into cytosol by sarcoplasmic reticulum",
  "gene_name": "Ryanodine receptor 2"
}